{
  "gene": "UniProtKB:Q05586",
  "term_label": "plasma membrane",
  "gene_symbol": "GRIN1",
  "term_id": "GO:0005886",
  "gene_name": "Glutamate receptor ionotropic, NMDA 1"
}